{
  "gene": "UniProtKB:Q99459",
  "term_id": "GO:0006357",
  "term_label": "regulation of transcription by RNA polymerase II",
  "gene_name": "Cell division cycle 5-like protein",
  "gene_symbol": "CDC5L"
}